central nervous system interneuron axonogenesis [GO:0021956] (biological process) Relationships: is a type of central nervous system neuron axonogenesis [GO:0021955] Definition: Generation of a long process that carries efferent (outgoing) action potentials from the cell body towards target cells from a neuron located in the central nervous system whose axons remain within a single brain region. Sources: GOC:cls, GOC:dgh, GOC:dph, GOC:jid, GO_REF:0000021